phosphatidylcholine catabolic process [GO:0034638] (biological process) Also known as: phosphatidylcholine breakdown, phosphatidylcholine catabolism, phosphatidylcholine degradation Sources: GOC:jp Definition: The chemical reactions and pathways resulting in the breakdown of phosphatidylcholines, any of a class of glycerophospholipids in which the phosphatidyl group is esterified to the hydroxyl group of choline. Relationships: is a type of phosphatidylcholine metabolic process [GO:0046470]; is a type of glycerophospholipid catabolic process [GO:0046475] Regulation: regulated by regulation of phosphatidylcholine catabolic process [GO:0010899]; negatively regulated by negative regulation of phosphatidylcholine catabolic process [GO:0010900]